{
  "gene_symbol": "PER3",
  "gene_name": "Period circadian protein homolog 3",
  "term_id": "GO:0005634",
  "term_label": "nucleus",
  "gene": "UniProtKB:P56645"
}